poly-N-acetyllactosamine metabolic process [GO:0030309] (biological process) Relationships: is a type of aminoglycan metabolic process [GO:0006022] Definition: The chemical reactions and pathways involving poly-N-acetyllactosamine, a carbohydrate composed of N-acetyllactosamine repeats (Gal-beta-1,4-GlcNAc-beta-1,3)n. References: PMID:9405606 Sources: GOC:mah Subtypes: poly-N-acetyllactosamine catabolic process [GO:0030310], poly-N-acetyllactosamine biosynthetic process [GO:0030311] Also known as: poly-N-acetyllactosamine metabolism